{
  "gene_symbol": "NR4A2",
  "gene": "UniProtKB:P43354",
  "gene_name": "Nuclear receptor subfamily 4 group A member 2",
  "term_label": "DNA-binding transcription factor activity, RNA polymerase II-specific",
  "term_id": "GO:0000981"
}